excitatory synapse [GO:0060076] (cellular component) Definition: A synapse in which an action potential in the presynaptic cell increases the probability of an action potential occurring in the postsynaptic cell. Relationships: is a type of synapse [GO:0045202] Subtypes: excitatory neuromuscular junction [GO:0098520], GO:0098688, asymmetric, glutamatergic, excitatory synapse [GO:0098985] Sources: GOC:dph, GOC:ef